protein-N(PI)-phosphohistidine-sugar phosphotransferase activity [GO:0008982] (molecular function) Subtypes: GO:0022855, protein-N(PI)-phosphohistidine-sorbitol phosphotransferase system transporter activity [GO:0022856], GO:0022869, protein-N(PI)-phosphohistidine-mannose phosphotransferase system transporter activity [GO:0022870], protein-N(PI)-phosphohistidine-sorbose phosphotransferase system transporter activity [GO:0022871], protein-N(PI)-phosphohistidine-mannitol phosphotransferase system transmembrane transporter activity [GO:0022872], protein-N(PI)-phosphohistidine-maltose phosphotransferase system transporter activity [GO:0022873], protein-N(PI)-phosphohistidine-cellobiose phosphotransferase system transporter activity [GO:0022874], protein-N(PI)-phosphohistidine-galactitol phosphotransferase system transmembrane transporter activity [GO:0022875], protein-N(PI)-phosphohistidine-galactosamine phosphotransferase system transporter activity [GO:0022876], GO:0022877, protein-N(PI)-phosphohistidine-sucrose phosphotransferase system transporter activity [GO:0022878], GO:0022879, protein-N(PI)-phosphohistidine-N-acetylglucosamine phosphotransferase system transporter activity [GO:0022880], protein-N(PI)-phosphohistidine-N-acetylgalactosamine phosphotransferase system transporter activity [GO:0022881], protein-N(PI)-phosphohistidine-beta-glucoside phosphotransferase system transporter activity [GO:0022882], GO:0090562, GO:0090590, protein-N(PI)-phosphohistidine-N-acetyl-mannosamine phosphotransferase system transporter activity [GO:0090591] Sources: GOC:mtg_transport, ISBN:0815340729 Definition: Catalysis of the PEP-dependent, phosphoryl transfer-driven transport of substances across a membrane. The transport happens by catalysis of the reaction: protein N-phosphohistidine + sugar(out) = protein histidine + sugar phosphate(in). This differs from primary and secondary active transport in that the solute is modified during transport. Also known as: phosphotransfer-driven group translocator, PEP--sugar phosphotransferase enzyme II activity, protein-Np-phosphohistidine-sugar phosphotransferase activity, PEP-dependent phosphotransferase enzyme II, PTS permease activity, PTS transporter, enzyme II of the phosphotransferase system, phosphoenolpyruvate-sugar phosphotransferase enzyme II, phosphohistidinoprotein-hexose phosphotransferase activity, phosphoprotein factor-hexose phosophotransferase activity Relationships: is a type of carbohydrate transmembrane transporter activity [GO:0015144]; is a type of phosphotransferase activity, alcohol group as acceptor [GO:0016773]; is a type of active transmembrane transporter activity [GO:0022804]